{
  "term_id": "GO:0033344",
  "gene": "UniProtKB:Q8IZY2",
  "term_label": "cholesterol efflux",
  "gene_symbol": "ABCA7",
  "gene_name": "Phospholipid-transporting ATPase ABCA7"
}